{
  "gene": "UniProtKB:P20783",
  "term_label": "negative regulation of neuron apoptotic process",
  "term_id": "GO:0043524",
  "gene_symbol": "NTF3",
  "gene_name": "Neurotrophin-3"
}